{
  "gene_symbol": "MENT",
  "gene": "UniProtKB:Q9BUN1",
  "term_id": "UNKNOWN:0001",
  "gene_name": "Protein MENT",
  "term_label": "Unknown molecular function"
}